quinate 3-dehydrogenase (NAD+) activity [GO:0030266] (molecular function) Definition: Catalysis of the reaction: (-)-quinate + NAD+ = (-)-3-dehydroquinate + NADH + H+. Sources: EC:1.1.1.24 Also known as: quinic dehydrogenase activity, quinate:NAD 3-oxidoreductase activity, quinate:NAD(+) 3-oxidoreductase activity, quinate:NAD 5-oxidoreductase activity, quinate:NAD(+) 5-oxidoreductase activity Relationships: is a type of oxidoreductase activity, acting on the CH-OH group of donors, NAD or NADP as acceptor [GO:0016616]